{
  "gene_symbol": "ALK",
  "term_id": "GO:0042127",
  "gene": "UniProtKB:Q9UM73",
  "term_label": "regulation of cell population proliferation",
  "gene_name": "ALK tyrosine kinase receptor"
}